positive regulation of bicoid mRNA localization [GO:0045854] (biological process) Also known as: positive regulation of bicoid mRNA localisation, up regulation of bicoid mRNA localization, up-regulation of bicoid mRNA localization, upregulation of bicoid mRNA localization, activation of bicoid mRNA localization, stimulation of bicoid mRNA localization Relationships: is_a regulation of bicoid mRNA localization [GO:0008359]; is a type of positive regulation of cell maturation [GO:1903431]; is a type of GO:1904582; positively regulates bicoid mRNA localization [GO:0045450] Sources: GOC:go_curators Definition: Any process that activates or increases the frequency, rate or extent of the process in which bicoid mRNA is transported to, or maintained in, a specific location.